RNA N6-methyladenosine methyltransferase complex [GO:0036396] (cellular component) Also known as: Mum2, Ime4, and Slz1 complex, WMM complex, METTL3-METTL14-WTAP methyltransferase complex, MIS complex, m(6)A writer complex, m6A methyltransferase complex References: PMID:22685417, PMID:24316715, PMID:24407421, PMID:29507755, PMID:29535189, PMID:29547716 Sources: GOC:dgf, GOC:sp Relationships: is a type of methyltransferase complex [GO:0034708] Definition: A RNA methyltransferase complex that catalyzes the post-transcriptional methylation of adenosine to form N6-methyladenosine (m6A). In budding yeast, the MIS complex consists of Mum2p, Ime4p and Slz1p. In vertebrates, the complex consists of METTL3, METTL14 and associated components WTAP, ZC3H13, VIRMA, CBLL1/HAKAI and in some cases of RBM15 (RBM15 or RBM15B).